negative regulation of mitochondrial membrane permeability involved in apoptotic process [GO:1902109] (biological process) Relationships: is_a negative regulation of mitochondrial membrane permeability [GO:0035795]; is a type of regulation of mitochondrial membrane permeability involved in apoptotic process [GO:1902108] Definition: Any negative regulation of mitochondrial membrane permeability that is involved in apoptotic process. References: PMID:19168129 Sources: GOC:TermGenie, GOC:mtg_apoptosis, GOC:pm Also known as: negative regulation of mitochondrial membrane permeability involved in apoptotic cell death, negative regulation of mitochondrial membrane permeability involved in apoptotic programmed cell death, negative regulation of mitochondrial membrane permeability involved in programmed cell death by apoptosis, negative regulation of transport across mitochondrial membrane involved in apoptotic cell death, negative regulation of transport across mitochondrial membrane involved in apoptotic process, negative regulation of transport across mitochondrial membrane involved in apoptotic programmed cell death, negative regulation of transport across mitochondrial membrane involved in programmed cell death by apoptosis, mitochondrial membrane impermeabilization involved in apoptosis, mitochondrial membrane impermeabilization involved in apoptotic cell death, mitochondrial membrane impermeabilization involved in apoptotic process, mitochondrial membrane impermeabilization involved in apoptotic program, mitochondrial membrane impermeabilization involved in apoptotic programmed cell death, mitochondrial membrane impermeabilization involved in programmed cell death by apoptosis, mitochondrial membrane impermeabilization involved in type I programmed cell death, negative regulation of mitochondrial membrane permeability involved in apoptosis, negative regulation of mitochondrial membrane permeability involved in apoptotic program, negative regulation of mitochondrial membrane permeability involved in type I programmed cell death, negative regulation of transport across mitochondrial membrane involved in apoptosis, negative regulation of transport across mitochondrial membrane involved in apoptotic program, negative regulation of transport across mitochondrial membrane involved in type I programmed cell death, mitochondrial membrane impermeability involved in apoptosis, mitochondrial membrane impermeability involved in apoptotic cell death, mitochondrial membrane impermeability involved in apoptotic process, mitochondrial membrane impermeability involved in apoptotic program, mitochondrial membrane impermeability involved in apoptotic programmed cell death, mitochondrial membrane impermeability involved in programmed cell death by apoptosis, mitochondrial membrane impermeability involved in signaling (initiator) caspase activity, mitochondrial membrane impermeability involved in type I programmed cell death, mitochondrial membrane impermeabilization involved in signaling (initiator) caspase activity, negative regulation of mitochondrial membrane permeability involved in signaling (initiator) caspase activity, negative regulation of transport across mitochondrial membrane involved in signaling (initiator) caspase activity